{
  "term_label": "telomeric DNA binding",
  "term_id": "GO:0042162",
  "gene_symbol": "RPA2",
  "gene": "UniProtKB:P15927",
  "gene_name": "Replication protein A 32 kDa subunit"
}